phagosome acidification [GO:0090383] (biological process) Sources: GOC:kmv, GOC:tb Relationships: is a type of intracellular pH reduction [GO:0051452]; BFO_0000050 phagosome maturation [GO:0090382] Also known as: phagosomal acidification Definition: Any process that reduces the pH of the phagosome, measured by the concentration of the hydrogen ion. Subtypes: GO:0090390